{
  "gene_symbol": "ZSCAN5DP",
  "gene_name": "Putative zinc finger and SCAN domain-containing protein 5D",
  "term_id": "UNKNOWN:0003",
  "gene": "UniProtKB:P0CG00",
  "term_label": "Unknown cellular component"
}